{
  "gene_symbol": "MAGEA2B",
  "term_id": "GO:0005634",
  "gene_name": "Melanoma-associated antigen 2",
  "gene": "UniProtKB:P43356",
  "term_label": "nucleus"
}